{
  "gene_symbol": "INHBB",
  "term_id": "GO:0007178",
  "gene_name": "Inhibin beta B chain",
  "gene": "UniProtKB:P09529",
  "term_label": "cell surface receptor protein serine/threonine kinase signaling pathway"
}